{
  "term_id": "GO:0070828",
  "term_label": "heterochromatin organization",
  "gene": "UniProtKB:Q96T68",
  "gene_symbol": "SETDB2",
  "gene_name": "Histone-lysine N-methyltransferase SETDB2"
}